{
  "gene_symbol": "RRAGD",
  "term_label": "GTPase activity",
  "gene": "UniProtKB:Q9NQL2",
  "gene_name": "Ras-related GTP-binding protein D",
  "term_id": "GO:0003924"
}